{
  "gene_symbol": "DEFB128",
  "gene_name": "Beta-defensin 128",
  "gene": "UniProtKB:Q7Z7B8",
  "term_label": "Unknown cellular component",
  "term_id": "UNKNOWN:0003"
}